{
  "term_id": "GO:0005737",
  "gene": "UniProtKB:Q15831",
  "gene_symbol": "STK11",
  "gene_name": "Serine_threonine-protein kinase STK11",
  "term_label": "cytoplasm"
}